{
  "gene_symbol": "GSDMA",
  "term_id": "GO:0001786",
  "term_label": "phosphatidylserine binding",
  "gene_name": "Gasdermin-A",
  "gene": "UniProtKB:Q96QA5"
}